{
  "term_id": "GO:0016020",
  "term_label": "membrane",
  "gene": "UniProtKB:Q3KNS1",
  "gene_name": "Patched domain-containing protein 3",
  "gene_symbol": "PTCHD3"
}